negative regulation of skeletal muscle satellite cell activation involved in skeletal muscle regeneration [GO:1901667] (biological process) Relationships: is a type of GO:0014717; is a type of negative regulation of skeletal muscle tissue regeneration [GO:0043417]; is_a negative regulation of cell activation [GO:0050866]; negatively regulates GO:0014901 Also known as: down regulation of satellite cell activation involved in skeletal muscle regeneration, down-regulation of satellite cell activation involved in skeletal muscle regeneration, downregulation of satellite cell activation involved in skeletal muscle regeneration, inhibition of satellite cell activation involved in skeletal muscle regeneration Definition: Any process that stops, prevents or reduces the frequency, rate or extent of satellite cell activation involved in skeletal muscle regeneration. References: PMID:21272575 Sources: GOC:TermGenie, GOC:dph